{
  "term_id": "UNKNOWN:0002",
  "term_label": "Unknown biological process",
  "gene": "UniProtKB:P0CW24",
  "gene_symbol": "PNMA6A",
  "gene_name": "Paraneoplastic antigen-like protein 6A"
}